{
  "term_id": "GO:0033550",
  "term_label": "MAP kinase tyrosine phosphatase activity",
  "gene_name": "Dual specificity protein phosphatase 7",
  "gene_symbol": "DUSP7",
  "gene": "UniProtKB:Q16829"
}